{
  "gene": "UniProtKB:P08134",
  "term_label": "mitotic cytokinesis",
  "term_id": "GO:0000281",
  "gene_symbol": "RHOC",
  "gene_name": "Rho-related GTP-binding protein RhoC"
}